{
  "gene_symbol": "MBLAC1",
  "gene_name": "Metallo-beta-lactamase domain-containing protein 1",
  "term_label": "Unknown cellular component",
  "gene": "UniProtKB:A4D2B0",
  "term_id": "UNKNOWN:0003"
}